protein-containing complex destabilizing activity [GO:0140776] (molecular function) Definition: A molecular function that involves direct binding to one of the subunits of a protein-containing complex and promoting the dissociation of one or many subunits. This often happens by changing the conformation of the protein being bound, which decreases its affinity for the rest of the complex. Relationships: is a type of molecular_function [GO:0003674] Subtypes: actin filament severing activity [GO:0003789], GO:0140545, actin filament debranching activity [GO:0140775], microtubule destabilizing activity [GO:0170060] Also known as: protein unfoldase activity References: PMID:23727094, PMID:29779865, PMID:34836783